{
  "gene": "UniProtKB:O43711",
  "term_id": "GO:0000981",
  "gene_symbol": "TLX3",
  "term_label": "DNA-binding transcription factor activity, RNA polymerase II-specific",
  "gene_name": "T-cell leukemia homeobox protein 3"
}